{
  "term_label": "Unknown cellular component",
  "term_id": "UNKNOWN:0003",
  "gene_symbol": "KRTAP5-7",
  "gene": "UniProtKB:Q6L8G8",
  "gene_name": "Keratin-associated protein 5-7"
}